{
  "gene_symbol": "MCCD1",
  "gene": "UniProtKB:P59942",
  "term_id": "UNKNOWN:0002",
  "gene_name": "Mitochondrial coiled-coil domain protein 1",
  "term_label": "Unknown biological process"
}